{
  "term_label": "intracellular signal transduction",
  "term_id": "GO:0035556",
  "gene_name": "Serine_threonine-protein kinase PAK 2",
  "gene": "UniProtKB:Q13177",
  "gene_symbol": "PAK2"
}